adenosine 5'-(hexahydrogen pentaphosphate) catabolic process [GO:1901911] (biological process) Also known as: adenosine 5'-(hexahydrogen pentaphosphate) breakdown, adenosine 5'-(hexahydrogen pentaphosphate) catabolism, adenosine 5'-(hexahydrogen pentaphosphate) degradation Relationships: is a type of purine ribonucleotide catabolic process [GO:0009154] References: PMID:10090752 Sources: GOC:TermGenie Definition: The chemical reactions and pathways resulting in the breakdown of adenosine 5'-(hexahydrogen pentaphosphate).